{
  "term_label": "Fanconi anaemia nuclear complex",
  "gene_name": "Centromere protein S",
  "gene": "UniProtKB:Q8N2Z9",
  "term_id": "GO:0043240",
  "gene_symbol": "CENPS"
}